{
  "gene_symbol": "EHBP1",
  "gene_name": "EH domain-binding protein 1",
  "term_id": "GO:0051015",
  "term_label": "actin filament binding",
  "gene": "UniProtKB:Q8NDI1"
}